{
  "gene_name": "Regulator of G-protein signaling 8",
  "term_id": "GO:0045744",
  "gene_symbol": "RGS8",
  "gene": "UniProtKB:P57771",
  "term_label": "negative regulation of G protein-coupled receptor signaling pathway"
}